{
  "gene_name": "Thioredoxin reductase 2, mitochondrial",
  "gene": "UniProtKB:Q9NNW7",
  "term_id": "GO:0005829",
  "term_label": "cytosol",
  "gene_symbol": "TXNRD2"
}